{
  "gene_symbol": "FGF6",
  "term_id": "GO:0022008",
  "gene": "UniProtKB:P10767",
  "term_label": "neurogenesis",
  "gene_name": "Fibroblast growth factor 6"
}